{
  "gene_name": "Radixin",
  "gene": "UniProtKB:P35241",
  "gene_symbol": "RDX",
  "term_label": "positive regulation of early endosome to late endosome transport",
  "term_id": "GO:2000643"
}